fatty acid derivative biosynthetic process [GO:1901570] (biological process) Definition: The chemical reactions and pathways resulting in the formation of fatty acid derivative. Subtypes: wax biosynthetic process [GO:0010025], diaminopimelate biosynthetic process [GO:0019877], GO:0036104, fatty-acyl-CoA biosynthetic process [GO:0046949], GO:0046951, fatty acid primary amide biosynthetic process [GO:0062112], leukotriene B4 biosynthetic process [GO:0097251], lovastatin biosynthetic process [GO:0140735], leukotriene D4 biosynthetic process [GO:1901750], leukotriene A4 biosynthetic process [GO:1901753], fatty acid methyl ester biosynthetic process [GO:1902899], fatty alcohol biosynthetic process [GO:1903175], GO:2001301 Also known as: fatty acid derivative anabolism, fatty acid derivative biosynthesis, fatty acid derivative formation, fatty acid derivative synthesis Sources: GOC:TermGenie, GOC:pr Relationships: is a type of lipid biosynthetic process [GO:0008610]; is a type of fatty acid derivative metabolic process [GO:1901568]